{
  "term_id": "GO:0005881",
  "term_label": "cytoplasmic microtubule",
  "gene": "UniProtKB:Q9H902",
  "gene_name": "Receptor expression-enhancing protein 1",
  "gene_symbol": "REEP1"
}